chloroplast thylakoid membrane [GO:0009535] (cellular component) Sources: GOC:lr, GOC:mtg_sensu Relationships: is a type of organelle outer membrane [GO:0031968]; is a type of plastid thylakoid membrane [GO:0055035]; is part of chloroplast thylakoid [GO:0009534] Definition: The pigmented membrane of a chloroplast thylakoid. An example of this component is found in Arabidopsis thaliana.